{
  "gene_name": "Chloride channel protein ClC-Ka",
  "gene": "UniProtKB:P51800",
  "term_label": "voltage-gated chloride channel activity",
  "term_id": "GO:0005247",
  "gene_symbol": "CLCNKA"
}